{
  "term_label": "Unknown cellular component",
  "term_id": "UNKNOWN:0003",
  "gene_name": "Olfactory receptor 4F21",
  "gene": "UniProtKB:O95013",
  "gene_symbol": "OR4F21"
}